{
  "gene": "UniProtKB:Q9H0M4",
  "gene_name": "Zinc finger CW-type PWWP domain protein 1",
  "gene_symbol": "ZCWPW1",
  "term_id": "UNKNOWN:0002",
  "term_label": "Unknown biological process"
}